regulation of transcription-coupled nucleotide-excision repair [GO:0090262] (biological process) Definition: Any process that modulates the frequency, rate, or extent of the nucleotide-excision repair process that carries out preferential repair of DNA lesions on the actively transcribed strand of the DNA duplex. In addition, the transcription-coupled nucleotide-excision repair pathway is required for the recognition and repair of a small subset of lesions that are not recognized by the global genome nucleotide excision repair pathway. Sources: GOC:tb Relationships: is a type of regulation of nucleotide-excision repair [GO:2000819]; regulates transcription-coupled nucleotide-excision repair [GO:0006283]